{
  "gene": "UniProtKB:Q6QAJ8",
  "gene_name": "Transmembrane protein 220",
  "term_id": "UNKNOWN:0001",
  "term_label": "Unknown molecular function",
  "gene_symbol": "TMEM220"
}